regulation of cardiac muscle tissue development [GO:0055024] (biological process) Also known as: regulation of heart muscle development Definition: Any process that modulates the frequency, rate or extent of cardiac muscle tissue development. Sources: GOC:vk Subtypes: positive regulation of cardiac muscle tissue development [GO:0055025], negative regulation of cardiac muscle tissue development [GO:0055026] Relationships: is a type of regulation of striated muscle tissue development [GO:0016202]; RO_0002211 cardiac muscle tissue development [GO:0048738]